{
  "gene": "UniProtKB:Q9NVS2",
  "term_id": "UNKNOWN:0002",
  "term_label": "Unknown biological process",
  "gene_symbol": "MRPS18A",
  "gene_name": "Large ribosomal subunit protein mL66"
}